{
  "gene_name": "Calcium_calmodulin-dependent protein kinase kinase 1",
  "gene_symbol": "CAMKK1",
  "term_id": "GO:0005737",
  "term_label": "cytoplasm",
  "gene": "UniProtKB:Q8N5S9"
}